trisaccharide transport [GO:2001088] (biological process) Sources: GOC:mengo_curators Relationships: is a type of oligosaccharide transport [GO:0015772] Subtypes: raffinose transport [GO:0015773], maltotriose transport [GO:2001089], maltotriulose transport [GO:2001090], GO:2001091, arabinotriose transport [GO:2001092], galactotriose transport [GO:2001093], xylotriose transport [GO:2001094], GO:2001095, cellotriose transport [GO:2001096], laminaritriose transport [GO:2001097] Definition: The directed movement of a trisaccharideacetate into, out of or within a cell, or between cells, by means of some agent such as a transporter or pore.